{
  "term_label": "Unknown molecular function",
  "gene": "UniProtKB:Q96CP2",
  "term_id": "UNKNOWN:0001",
  "gene_name": "FLYWCH family member 2",
  "gene_symbol": "FLYWCH2"
}